{
  "gene_symbol": "JAML",
  "gene_name": "Junctional adhesion molecule-like",
  "term_label": "monocyte extravasation",
  "term_id": "GO:0035696",
  "gene": "UniProtKB:Q86YT9"
}